nuclear inclusion body [GO:0042405] (cellular component) Definition: An intranuclear focus at which aggregated proteins have been sequestered. Relationships: is a type of inclusion body [GO:0016234]; is part of nucleus [GO:0005634] Sources: GOC:jl Subtypes: nucleolar peripheral inclusion body [GO:0140602]